pilus retraction [GO:0043108] (biological process) References: PMID:17355871 Sources: GOC:go_curators Relationships: is a type of GO:0043711 Definition: The process of withdrawing a pilus back into a cell.